{
  "gene": "UniProtKB:Q9NZJ5",
  "gene_name": "Eukaryotic translation initiation factor 2-alpha kinase 3",
  "term_id": "GO:0004694",
  "gene_symbol": "EIF2AK3",
  "term_label": "eukaryotic translation initiation factor 2alpha kinase activity"
}